oncostatin-M receptor activity [GO:0004924] (molecular function) Sources: GOC:mah, GOC:signaling Definition: Combining with oncostatin-M and transmitting the signal from one side of the membrane to the other to initiate a change in cell activity. Relationships: is a type of cytokine receptor activity [GO:0004896]; is part of oncostatin-M-mediated signaling pathway [GO:0038165]